{
  "gene_name": "Raftlin-2",
  "gene_symbol": "RFTN2",
  "term_id": "UNKNOWN:0003",
  "term_label": "Unknown cellular component",
  "gene": "UniProtKB:Q52LD8"
}